{
  "term_label": "Unknown molecular function",
  "gene": "UniProtKB:Q53H64",
  "gene_name": "Putative ANKRD40 C-terminal-like protein",
  "gene_symbol": "ANKRD40CL",
  "term_id": "UNKNOWN:0001"
}